acquisition of plant reproductive competence [GO:0010049] (BP) Also known as: acquisition of reproductive competence Relationships: is a type of GO:0009791 Definition: The process in which a plant acquires the ability to respond to a floral inductive signal. Sources: GOC:tair_curators